{
  "term_id": "GO:0070059",
  "gene_name": "Serine_threonine-protein kinase_endoribonuclease IRE1",
  "gene_symbol": "ERN1",
  "term_label": "intrinsic apoptotic signaling pathway in response to endoplasmic reticulum stress",
  "gene": "UniProtKB:O75460"
}